type IV pilus [GO:0044096] (cellular component) References: PMID:28496159 Sources: GOC:pamgo_curators Relationships: is a type of GO:0009289 Definition: A short filamentous structure on the surface of a bacterial cell distinguished from other pili by post-translational N-methylation of the pilin monomers. Also known as: TFP, type 4 pilus, type IV fimbriae